{
  "gene_symbol": "OR13H1",
  "term_id": "GO:0004984",
  "gene": "UniProtKB:Q8NG92",
  "term_label": "olfactory receptor activity",
  "gene_name": "Olfactory receptor 13H1"
}